{
  "gene_symbol": "STARD9",
  "term_id": "GO:0005737",
  "gene": "UniProtKB:Q9P2P6",
  "term_label": "cytoplasm",
  "gene_name": "StAR-related lipid transfer protein 9"
}